{
  "gene_symbol": "C1RL",
  "term_id": "GO:0072562",
  "term_label": "blood microparticle",
  "gene_name": "Complement C1r subcomponent-like protein",
  "gene": "UniProtKB:Q9NZP8"
}